endoplasmic reticulum-plasma membrane adaptor activity [GO:0160214] (molecular function) Relationships: is a type of protein-membrane adaptor activity [GO:0043495] References: PMID:23041194, PMID:39239853 Definition: The binding activity of a molecule that brings together a plasma membrane with an endoplasmic reticulum membrane, via membrane lipid binding, to establish membrane contact sites and mediate exchange and communication.